{
  "gene_name": "G patch domain-containing protein 2",
  "gene": "UniProtKB:Q9NW75",
  "term_label": "nucleus",
  "gene_symbol": "GPATCH2",
  "term_id": "GO:0005634"
}